{
  "gene_symbol": "CYP2W1",
  "gene": "UniProtKB:Q8TAV3",
  "gene_name": "Cytochrome P450 2W1",
  "term_label": "heme binding",
  "term_id": "GO:0020037"
}